skeletal system development [GO:0001501] (biological process) Definition: The process whose specific outcome is the progression of the skeleton over time, from its formation to the mature structure. The skeleton is the bony framework of the body in vertebrates (endoskeleton) or the hard outer envelope of insects (exoskeleton or dermoskeleton). Sources: GOC:dph, GOC:jid, GOC:tb Also known as: skeletal development Relationships: is_a GO:0048731 Subtypes: embryonic skeletal system development [GO:0048706]